{
  "term_id": "GO:0006325",
  "gene_name": "High mobility group nucleosome-binding domain-containing protein 3",
  "gene": "UniProtKB:Q15651",
  "gene_symbol": "HMGN3",
  "term_label": "chromatin organization"
}